{
  "term_label": "stress fiber",
  "gene_name": "PDZ and LIM domain protein 1",
  "gene": "UniProtKB:O00151",
  "term_id": "GO:0001725",
  "gene_symbol": "PDLIM1"
}